{
  "gene_symbol": "BAG5",
  "gene": "UniProtKB:Q9UL15",
  "term_id": "GO:0005737",
  "term_label": "cytoplasm",
  "gene_name": "BAG family molecular chaperone regulator 5"
}